mesonephric glomerulus development [GO:0061224] (biological process) Sources: GOC:mtg_kidney_jan10 Relationships: is a type of GO:0032835; BFO_0000050 mesonephric nephron development [GO:0061215] Definition: The progression of the mesonephric glomerulus over time from its initial formation until its mature state. The mesonephric glomerulus is a capillary tuft which forms a close network with the visceral epithelium (podocytes) and the mesangium to form the filtration barrier and is surrounded by Bowman's capsule in nephrons of the mature vertebrate kidney, or mesonephros. Regulation: regulated by regulation of mesonephric glomerulus development [GO:2000087]; negatively regulated by negative regulation of mesonephric glomerulus development [GO:2000088]; positively regulated by positive regulation of mesonephric glomerulus development [GO:2000089]